{
  "term_label": "protein folding",
  "gene_name": "Peptidyl-prolyl cis-trans isomerase A-like 4C",
  "term_id": "GO:0006457",
  "gene": "UniProtKB:A0A0B4J2A2",
  "gene_symbol": "PPIAL4C"
}